{
  "gene": "UniProtKB:P0DP72",
  "gene_symbol": "VSIG10L2",
  "gene_name": "V-set and immunoglobulin domain-containing protein 10-like 2",
  "term_label": "plasma membrane",
  "term_id": "GO:0005886"
}